{
  "term_id": "GO:0012506",
  "gene": "UniProtKB:P27216",
  "gene_name": "Annexin A13",
  "gene_symbol": "ANXA13",
  "term_label": "vesicle membrane"
}